{
  "term_id": "GO:0005886",
  "gene_name": "Cationic amino acid transporter 4",
  "gene_symbol": "SLC7A4",
  "gene": "UniProtKB:O43246",
  "term_label": "plasma membrane"
}